{
  "term_id": "UNKNOWN:0003",
  "term_label": "Unknown cellular component",
  "gene": "UniProtKB:Q9ULI4",
  "gene_symbol": "KIF26A",
  "gene_name": "Kinesin-like protein KIF26A"
}